{
  "gene": "UniProtKB:Q8N7G0",
  "term_id": "GO:0006357",
  "gene_symbol": "POU5F2",
  "term_label": "regulation of transcription by RNA polymerase II",
  "gene_name": "POU domain, class 5, transcription factor 2"
}